{
  "term_label": "GPI-anchor transamidase activity",
  "gene_name": "Phosphatidylinositol glycan anchor biosynthesis class U protein",
  "gene": "UniProtKB:Q9H490",
  "gene_symbol": "PIGU",
  "term_id": "GO:0003923"
}